{
  "gene_symbol": "RASGEF1A",
  "gene_name": "Ras-GEF domain-containing family member 1A",
  "gene": "UniProtKB:Q8N9B8",
  "term_id": "GO:0005085",
  "term_label": "guanyl-nucleotide exchange factor activity"
}